{
  "gene_symbol": "AMIGO3",
  "gene_name": "Amphoterin-induced protein 3",
  "term_id": "GO:0007157",
  "gene": "UniProtKB:Q86WK7",
  "term_label": "heterophilic cell-cell adhesion"
}